{
  "term_label": "replication fork arrest",
  "term_id": "GO:0043111",
  "gene_name": "TIMELESS-interacting protein",
  "gene_symbol": "TIPIN",
  "gene": "UniProtKB:Q9BVW5"
}